{
  "gene_name": "Interleukin-26",
  "gene": "UniProtKB:Q9NPH9",
  "gene_symbol": "IL26",
  "term_id": "GO:0005615",
  "term_label": "extracellular space"
}